{
  "gene_symbol": "MYO9B",
  "gene": "UniProtKB:Q13459",
  "term_id": "GO:0030048",
  "gene_name": "Unconventional myosin-IXb",
  "term_label": "actin filament-based movement"
}